cytoplasmic streaming [GO:0099636] (biological process) Relationships: is a type of intracellular transport [GO:0046907] Sources: GOC:dos, Wikipedia:Cytoplasmic_streaming&oldid=706214009 Definition: The directed flow of cytosol (the liquid component of the cytoplasm) and the organelles it contains.